{
  "term_label": "cytosolic large ribosomal subunit",
  "gene_symbol": "RPL17",
  "term_id": "GO:0022625",
  "gene": "UniProtKB:P18621",
  "gene_name": "Large ribosomal subunit protein uL22"
}